{
  "term_label": "tricarboxylic acid cycle",
  "gene": "UniProtKB:P48735",
  "gene_symbol": "IDH2",
  "term_id": "GO:0006099",
  "gene_name": "Isocitrate dehydrogenase [NADP], mitochondrial"
}